glycine N-benzoyltransferase activity [GO:0047962] (molecular function) Also known as: benzoyl CoA-amino acid N-acyltransferase activity, benzoyl-CoA:glycine N-acyltransferase activity, benzoyl-CoA:glycine N-benzoyltransferase activity Definition: Catalysis of the reaction: benzoyl-CoA + glycine = N-benzoylglycine + CoA + H+. Sources: EC:2.3.1.71, RHEA:18493 Relationships: is a type of acyltransferase activity, transferring groups other than amino-acyl groups [GO:0016747]